{
  "term_label": "extracellular space",
  "gene": "UniProtKB:Q6UW88",
  "term_id": "GO:0005615",
  "gene_symbol": "EPGN",
  "gene_name": "Epigen"
}